shamixanthone catabolic process [GO:1900792] (biological process) Sources: GOC:TermGenie, GOC:di Relationships: is a type of phenol-containing compound catabolic process [GO:0019336]; is a type of ketone catabolic process [GO:0042182]; is a type of GO:0090487 Also known as: shamixanthone breakdown, shamixanthone catabolism, shamixanthone degradation Definition: The chemical reactions and pathways resulting in the breakdown of shamixanthone.